{
  "term_id": "GO:0005829",
  "gene_name": "Transketolase-like protein 1",
  "term_label": "cytosol",
  "gene": "UniProtKB:P51854",
  "gene_symbol": "TKTL1"
}